{
  "term_label": "sodium channel regulator activity",
  "gene_name": "Fibroblast growth factor 14",
  "gene": "UniProtKB:Q92915",
  "gene_symbol": "FGF14",
  "term_id": "GO:0017080"
}